{
  "term_id": "GO:0007411",
  "gene_name": "Neuronal cell adhesion molecule",
  "gene_symbol": "NRCAM",
  "gene": "UniProtKB:Q92823",
  "term_label": "axon guidance"
}